granulocyte macrophage colony-stimulating factor receptor binding [GO:0005129] (molecular function) Also known as: GM-CSF receptor binding, granulocyte macrophage colony stimulating factor receptor binding, GM-CSF receptor ligand, GMC-SF receptor ligand, granulocyte macrophage colony-stimulating factor, granulocyte macrophage colony-stimulating factor receptor ligand Definition: Binding to a granulocyte macrophage colony-stimulating factor receptor. Relationships: is a type of cytokine receptor binding [GO:0005126]; is a type of growth factor receptor binding [GO:0070851] Sources: GOC:ai